{
  "gene_name": "Protein sidekick-2",
  "term_label": "Unknown molecular function",
  "gene": "UniProtKB:Q58EX2",
  "term_id": "UNKNOWN:0001",
  "gene_symbol": "SDK2"
}